{
  "gene": "UniProtKB:O14974",
  "term_id": "GO:0005737",
  "gene_name": "Protein phosphatase 1 regulatory subunit 12A",
  "gene_symbol": "PPP1R12A",
  "term_label": "cytoplasm"
}